L-ascorbic acid metabolic process [GO:0019852] (biological process) Sources: GOC:jl, ISBN:0198506732 Relationships: is a type of monosaccharide metabolic process [GO:0005996]; is a type of carboxylic acid metabolic process [GO:0019752]; is a type of lactone metabolic process [GO:1901334] Definition: The chemical reactions and pathways involving L-ascorbic acid, (2R)-2-[(1S)-1,2-dihydroxyethyl]-4-hydroxy-5-oxo-2,5-dihydrofuran-3-olate; L-ascorbic acid is vitamin C and has co-factor and anti-oxidant activities in many species. Also known as: L-ascorbic acid metabolism, ascorbate metabolic process, ascorbate metabolism, vitamin C metabolic process, vitamin C metabolism Subtypes: L-ascorbic acid biosynthetic process [GO:0019853], L-ascorbic acid catabolic process [GO:0019854], ascorbate glutathione cycle [GO:0033355]